{
  "gene_name": "Cytochrome P450 4A22",
  "term_label": "lauric acid metabolic process",
  "term_id": "GO:0048252",
  "gene": "UniProtKB:Q5TCH4",
  "gene_symbol": "CYP4A22"
}